androgen receptor signaling pathway [GO:0030521] (biological process) Relationships: is a type of GO:0030518 Also known as: androgen receptor signalling pathway, nuclear-receptor-mediated androgen receptor signaling pathway Regulation: regulated by regulation of androgen receptor signaling pathway [GO:0060765]; negatively regulated by negative regulation of androgen receptor signaling pathway [GO:0060766]; positively regulated by positive regulation of androgen receptor signaling pathway [GO:0160207] Sources: GOC:mah Definition: A nuclear receptor-mediated signaling pathway initiated by an androgen binding to an intracellular receptor of the nuclear receptor protein family, and ending with regulation of a downstream cellular process, e.g. transcription.